{
  "term_id": "GO:0005737",
  "gene_name": "Malate dehydrogenase, mitochondrial",
  "gene_symbol": "MDH2",
  "term_label": "cytoplasm",
  "gene": "UniProtKB:P40926"
}